regulation of ventricular cardiac muscle cell membrane repolarization [GO:0060307] (biological process) Definition: Any process that modulates the establishment or extent of a membrane potential in the polarizing direction towards the resting potential in a ventricular cardiomyocyte. Sources: GOC:BHF, GOC:dph, GOC:mtg_cardiac_conduct_nov11, GOC:tb Also known as: regulation of ventricular cardiac muscle cell repolarization, regulation of ventricular cardiomyocyte membrane repolarization, electrocardiogram T wave, regulation of ventricular cardiac muscle repolarization, ventricular repolarization Relationships: is a type of GO:0099623; regulates ventricular cardiac muscle cell membrane repolarization [GO:0099625] Subtypes: GO:1905024